{
  "gene_name": "Mothers against decapentaplegic homolog 1",
  "term_id": "GO:0071144",
  "gene_symbol": "SMAD1",
  "gene": "UniProtKB:Q15797",
  "term_label": "heteromeric SMAD protein complex"
}